{
  "gene": "UniProtKB:A6NEH6",
  "term_label": "Unknown biological process",
  "gene_symbol": "TMEM247",
  "gene_name": "Transmembrane protein 247",
  "term_id": "UNKNOWN:0002"
}